{
  "gene_symbol": "KLF14",
  "gene": "UniProtKB:Q8TD94",
  "term_label": "nucleus",
  "gene_name": "Krueppel-like factor 14",
  "term_id": "GO:0005634"
}